response to vanadate(3-) [GO:1902438] (biological process) References: PMID:7489911 Sources: GOC:TermGenie, GOC:di Relationships: is a type of response to oxygen-containing compound [GO:1901700] Subtypes: cellular response to vanadate(3-) [GO:1902439] Definition: Any process that results in a change in state or activity of a cell or an organism (in terms of movement, secretion, enzyme production, gene expression, etc.) as a result of a vanadate(3-) stimulus.